protein arginine N5-methyltransferase activity [GO:0019702] (molecular function) Relationships: is a type of protein-arginine N-methyltransferase activity [GO:0016274] References: PMID:11856739, PMID:9873020 Sources: EC:2.1.1.322 Also known as: protein arginine N5-methylase activity, protein-arginine N5-methyltransferase activity, protein-arginine delta-N-methyltransferase activity, type IV PRMT activity, type IV protein arginine methyltransferase activity, S-adenosyl-L-methionine:[protein]-L-arginine N-methyltransferase ([protein]-N5-methyl-L-arginine-forming) Note: This enzyme, characterized from the yeast Saccharomyces cerevisiae, methylates the delta-nitrogen atom of arginine residues within proteins. Among its substrates are R67 of the ribosomal protein L12. Definition: Catalysis of the transfer of a methyl group from S-adenosyl-L-methionine to the delta-nitrogen atom of peptidyl-arginine residues. The reaction is S-adenosyl-L-methionine + [protein]-L-arginine = S-adenosyl-L-homocysteine + [protein]-N5-methyl-L-arginine.